{
  "gene_name": "Mitochondrial enolase superfamily member 1",
  "term_label": "magnesium ion binding",
  "term_id": "GO:0000287",
  "gene_symbol": "ENOSF1",
  "gene": "UniProtKB:Q7L5Y1"
}